{
  "gene": "UniProtKB:P22888",
  "term_label": "luteinizing hormone receptor activity",
  "term_id": "GO:0004964",
  "gene_name": "Lutropin-choriogonadotropic hormone receptor",
  "gene_symbol": "LHCGR"
}